polyphosphate biosynthetic process [GO:0006799] (BP) Relationships: is a type of GO:0006797; is a type of GO:0009058 Definition: The chemical reactions and pathways resulting in the formation of a polyphosphate, the anion or salt of polyphosphoric acid. Sources: ISBN:0198506732 Also known as: polyphosphate anabolism, polyphosphate biosynthesis, polyphosphate formation, polyphosphate synthesis